{
  "gene_symbol": "SERPINA2",
  "term_id": "UNKNOWN:0002",
  "term_label": "Unknown biological process",
  "gene_name": "Alpha-1-antitrypsin-related protein",
  "gene": "UniProtKB:P20848"
}